{
  "gene_symbol": "TRMT6",
  "term_id": "UNKNOWN:0002",
  "gene_name": "tRNA (adenine(58)-N(1))-methyltransferase non-catalytic subunit TRM6",
  "term_label": "Unknown biological process",
  "gene": "UniProtKB:Q9UJA5"
}